{
  "gene": "UniProtKB:P12643",
  "term_label": "BMP signaling pathway",
  "term_id": "GO:0030509",
  "gene_symbol": "BMP2",
  "gene_name": "Bone morphogenetic protein 2"
}